{
  "gene": "UniProtKB:Q8NEG2",
  "gene_name": "Uncharacterized protein C7orf57",
  "gene_symbol": "C7orf57",
  "term_id": "UNKNOWN:0001",
  "term_label": "Unknown molecular function"
}